{
  "gene_name": "Insulin-induced gene 1 protein",
  "term_label": "SREBP-SCAP complex retention in endoplasmic reticulum",
  "gene": "UniProtKB:O15503",
  "gene_symbol": "INSIG1",
  "term_id": "GO:0036316"
}